{
  "gene_name": "Histone demethylase UTY",
  "term_label": "histone H3K27me2/H3K27me3 demethylase activity",
  "gene_symbol": "UTY",
  "gene": "UniProtKB:O14607",
  "term_id": "GO:0071558"
}